insulin-like growth factor binary complex [GO:0042568] (cellular component) Also known as: IGF binary complex Definition: A complex of two proteins, which in animals is 50kDa and consists of the insulin-like growth factor (IGF) and one of the insulin-like growth factor binding protein-1 (IGFBP-1), -2 (IGFBP-2), -4 (IGFBP-4) and -6 (IGFBP-6). The complex plays a role in growth and development. References: PMID:12239079 Sources: GOC:jl Relationships: is a type of GO:0016942